G-protein beta/gamma-Raf-1 complex [GO:0070422] (cellular component) Note: See also the cellular component term 'heterotrimeric G-protein complex ; GO:0005834'. Definition: A protein complex formed by the association of the serine-threonine protein kinase Raf-1 with the beta and gamma subunits of a heterotrimeric G protein. References: PMID:7782277 Sources: GOC:mah Relationships: is a type of protein-containing complex [GO:0032991]; is part of cytoplasm [GO:0005737] Also known as: G protein complex (GNG2, GNB2L1, RAF1)